ligand-gated ion channel signaling pathway [GO:1990806] (biological process) References: PMID:25869137 Sources: GOC:bhm Subtypes: ionotropic glutamate receptor signaling pathway [GO:0035235], GO:0140227 Definition: The series of molecular signals initiated by activation of a ligand-gated ion channel on the surface of a cell. The pathway begins with binding of an extracellular ligand to a ligand-gated ion channel and ends with a molecular function that directly regulates a downstream cellular process, e.g. transcription. Also known as: ligand-gated ion channel signalling pathway Relationships: is a type of GO:0007165; has part ligand-gated monoatomic ion channel activity [GO:0015276]